{
  "gene_symbol": "NEDD4",
  "gene": "UniProtKB:P46934",
  "gene_name": "E3 ubiquitin-protein ligase NEDD4",
  "term_id": "GO:0050807",
  "term_label": "regulation of synapse organization"
}